protein-phosphocysteine-N-acetylmuramate phosphotransferase system transporter activity [GO:0090588] (molecular function) References: PMID:15060041 Relationships: is a type of protein-phosphocysteine-sugar phosphotransferase activity [GO:0090563] Definition: Catalysis of the PEP-dependent, phosphoryl transfer-driven transport of substances across a membrane. The transport happens by catalysis of the reaction: protein S-phosphocysteine + N-acetylmuramate (out) = protein cysteine + N-acetylmuramate-6-phosphate (in).